{
  "term_label": "dynein intermediate chain binding",
  "gene_symbol": "DNAH11",
  "gene_name": "Dynein axonemal heavy chain 11",
  "term_id": "GO:0045505",
  "gene": "UniProtKB:Q96DT5"
}